{
  "term_label": "regulation of transcription by RNA polymerase II",
  "term_id": "GO:0006357",
  "gene": "UniProtKB:P81133",
  "gene_symbol": "SIM1",
  "gene_name": "Single-minded homolog 1"
}